{
  "gene_name": "Leiomodin-2",
  "gene": "UniProtKB:Q6P5Q4",
  "term_label": "myofibril assembly",
  "term_id": "GO:0030239",
  "gene_symbol": "LMOD2"
}